{
  "gene_name": "Interferon-induced GTP-binding protein Mx2",
  "term_label": "synaptic vesicle budding from presynaptic endocytic zone membrane",
  "term_id": "GO:0016185",
  "gene_symbol": "MX2",
  "gene": "UniProtKB:P20592"
}